{
  "term_id": "GO:0000978",
  "gene": "UniProtKB:O60304",
  "gene_name": "Zinc finger protein 500",
  "gene_symbol": "ZNF500",
  "term_label": "RNA polymerase II cis-regulatory region sequence-specific DNA binding"
}